{
  "gene_symbol": "C6orf118",
  "term_id": "UNKNOWN:0003",
  "gene_name": "Uncharacterized protein C6orf118",
  "term_label": "Unknown cellular component",
  "gene": "UniProtKB:Q5T5N4"
}